glucuronyl-galactosyl-proteoglycan 4-alpha-N-acetylglucosaminyltransferase activity [GO:0001888] (molecular function) Sources: EC:2.4.1.223, RHEA:16221 Relationships: is a type of GO:0008375 Definition: Catalysis of the reaction: 3-O-(beta-D-GlcA-(1->3)-beta-D-Gal-(1->3)-beta-D-Gal-(1->4)-beta-D-Xyl)-L-seryl-[protein] + UDP-N-acetyl-alpha-D-glucosamine = 3-O-(alpha-D-GlcNAc-(1->4)-beta-D-GlcA-(1->3)-beta-D-Gal-(1->3)-beta-D-Gal-(1->4)-beta-D-Xyl)-L-seryl-[protein] + H+ + UDP. Also known as: UDP-N-acetyl-D-glucosamine:beta-D-glucuronosyl-(1,3)-beta-D-galactosyl-(1,3)-beta-D-galactosyl-(1,4)-beta-D-xylosyl-proteoglycan 4IV-alpha-N-acetyl-D-glucosaminyltransferase activity, UDP-N-acetyl-D-glucosamine:beta-D-glucuronosyl-(1->3)-beta-D-galactosyl-(1->3)-beta-D-galactosyl-(1->4)-beta-D-xylosyl-proteoglycan 4IV-alpha-N-acetyl-D-glucosaminyltransferase activity, alpha-1,4-N-acetylglucosaminyltransferase activity, alpha-N-acetylglucosaminyltransferase I activity, alpha1,4-N-acetylglucosaminyltransferase activity, glucuronosylgalactosyl-proteoglycan 4-alpha-N-acetylglucosaminyltransferase activity